oligopeptide transmembrane transporter activity [GO:0035673] (molecular function) Relationships: is a type of amide transmembrane transporter activity [GO:0042887]; BFO_0000050 oligopeptide transmembrane transport [GO:0035672] Definition: Enables the transfer of oligopeptides from one side of a membrane to the other. Oligopeptides are molecules that contain a small number (2 to 20) of amino-acid residues connected by peptide linkages. Also known as: oligopeptide transporter activity Sources: GOC:vw, ISBN:0198506732 Subtypes: high-affinity oligopeptide transmembrane transporter activity [GO:0015334], ABC-type oligopeptide transporter activity [GO:0015421], tripeptide transmembrane transporter activity [GO:0042937], dipeptide transmembrane transporter activity [GO:0071916], tetrapeptide transmembrane transporter activity [GO:1901584]